{
  "term_id": "GO:0050585",
  "gene_name": "4-hydroxyphenylpyruvate dioxygenase-like protein",
  "gene_symbol": "HPDL",
  "term_label": "4-hydroxymandelate synthase activity",
  "gene": "UniProtKB:Q96IR7"
}